{
  "gene": "UniProtKB:Q9NZK5",
  "gene_name": "Adenosine deaminase 2",
  "gene_symbol": "ADA2",
  "term_label": "adenosine catabolic process",
  "term_id": "GO:0006154"
}